{
  "gene": "UniProtKB:Q10571",
  "term_id": "UNKNOWN:0001",
  "gene_name": "Transcriptional activator MN1",
  "term_label": "Unknown molecular function",
  "gene_symbol": "MN1"
}